{
  "gene": "UniProtKB:A0A075B6W5",
  "gene_name": "T cell receptor alpha variable 23_delta variable 6",
  "term_label": "peptide antigen binding",
  "term_id": "GO:0042605",
  "gene_symbol": "TRAV23DV6"
}